juvenile hormone catabolic process [GO:0006719] (biological process) Definition: The chemical reactions and pathways resulting in the breakdown of juvenile hormones, the three sesquiterpenoid derivatives that function to maintain the larval state of insects at molting and that may be required for other processes, e.g. oogenesis. Regulation: regulated by regulation of juvenile hormone catabolic process [GO:0045952]; negatively regulated by GO:0045970; positively regulated by GO:0045971 Relationships: is a type of juvenile hormone metabolic process [GO:0006716]; is a type of sesquiterpenoid catabolic process [GO:0016107]; is a type of hormone catabolic process [GO:0042447] Also known as: juvenile hormone breakdown, juvenile hormone catabolism, juvenile hormone degradation Sources: GOC:go_curators, ISBN:0198547684